{
  "gene_symbol": "MTX1",
  "term_id": "UNKNOWN:0001",
  "term_label": "Unknown molecular function",
  "gene_name": "Metaxin-1",
  "gene": "UniProtKB:Q13505"
}